somatic recombination of T cell receptor gene segments [GO:0002681] (biological process) Sources: GOC:add, ISBN:0781735149 Also known as: somatic recombination of TCR gene segments Subtypes: GO:0033153 Definition: The process in which T cell receptor genes are formed through recombination of the germline genetic elements, also known as T cell receptor gene segments. Relationships: is a type of somatic diversification of immune receptors via germline recombination within a single locus [GO:0002562]; is a type of somatic diversification of T cell receptor genes [GO:0002568]